negative regulation of double-strand break repair via homologous recombination [GO:2000042] (biological process) Definition: Any process that stops, prevents, or reduces the frequency, rate or extent of double-strand break repair via homologous recombination. Sources: GOC:vw Also known as: negative regulation of HDR, negative regulation of HRR, negative regulation of Rad51-dependent recombinational repair, negative regulation of Rhp51-dependent recombinational repair, negative regulation of homologous recombinational repair, negative regulation of homology-directed repair Relationships: is a type of GO:0010569; is a type of negative regulation of DNA recombination [GO:0045910]; is a type of negative regulation of double-strand break repair [GO:2000780]; negatively regulates double-strand break repair via homologous recombination [GO:0000724] Subtypes: negative regulation of double-strand break repair via break-induced replication [GO:1901592]